{
  "term_label": "Unknown cellular component",
  "term_id": "UNKNOWN:0003",
  "gene_name": "Dynein axonemal assembly factor 4",
  "gene_symbol": "DNAAF4",
  "gene": "UniProtKB:Q8WXU2"
}